modified histidine biosynthetic process [GO:0052703] (biological process) Definition: The chemical reactions and pathways resulting in the formation of compounds derived from histidine, 2-amino-3-(1H-imidazol-4-yl)propanoic acid within a cell. Also known as: cellular histidine derivative anabolism, cellular histidine derivative biosynthesis, cellular histidine derivative biosynthetic process, cellular histidine derivative formation, cellular histidine derivative synthesis, cellular modified histidine anabolism, cellular modified histidine biosynthesis, cellular modified histidine formation, cellular modified histidine synthesis, histidine derivative biosynthetic process Subtypes: GO:0052699, selenoneine biosynthetic process [GO:1903257] Relationships: is a type of modified amino acid biosynthetic process [GO:0042398] Sources: GOC:ai